{
  "term_id": "GO:0006508",
  "gene_symbol": "LVRN",
  "gene": "UniProtKB:Q6Q4G3",
  "term_label": "proteolysis",
  "gene_name": "Aminopeptidase Q"
}